{
  "gene_name": "E3 ubiquitin-protein ligase parkin",
  "gene_symbol": "PRKN",
  "term_label": "cytosol",
  "term_id": "GO:0005829",
  "gene": "UniProtKB:O60260"
}